{
  "term_label": "regulation of synaptic plasticity",
  "gene": "UniProtKB:O15240",
  "gene_symbol": "VGF",
  "gene_name": "Neurosecretory protein VGF",
  "term_id": "GO:0048167"
}